Hrd1p ubiquitin ligase ERAD-M complex [GO:0000838] (cellular component) References: PMID:16873066 Sources: GOC:elh Definition: A multiprotein complex that recognizes and ubiquitinates proteins with misfolded membrane domains during ER-associated protein degradation (ERAD). In S. cerevisiae, this complex contains the ubiquitin ligase Hrd1p. Relationships: is a type of GO:0000836